negative regulation of bone mineralization involved in bone maturation [GO:1900158] (BP) Definition: Any process that stops, prevents or reduces the frequency, rate or extent of bone mineralization involved in bone maturation. Sources: GOC:BHF, GOC:TermGenie Also known as: down regulation of bone mineralization involved in bone maturation, down-regulation of bone mineralization involved in bone maturation, downregulation of bone mineralization involved in bone maturation, inhibition of bone mineralization involved in bone maturation Relationships: is a type of negative regulation of bone mineralization [GO:0030502]; is a type of GO:1900157; negatively regulates bone mineralization involved in bone maturation [GO:0035630]